{
  "term_id": "UNKNOWN:0002",
  "gene_symbol": "OR4K2",
  "term_label": "Unknown biological process",
  "gene": "UniProtKB:Q8NGD2",
  "gene_name": "Olfactory receptor 4K2"
}